{
  "term_id": "GO:0005687",
  "gene_symbol": "SNRPD1",
  "term_label": "U4 snRNP",
  "gene_name": "Small nuclear ribonucleoprotein Sm D1",
  "gene": "UniProtKB:P62314"
}